glycerol 2-dehydrogenase (NADP+) activity [GO:0047953] (molecular function) Definition: Catalysis of the reaction: glycerol + NADP+ = dihydroxyacetone + NADPH + H+. Also known as: DHA oxidoreductase activity, dihydroxyacetone (reduced nicotinamide adenine dinucleotide phosphate) reductase activity, dihydroxyacetone reductase (NADPH), dihydroxyacetone reductase activity, glycerol:NADP+ 2-oxidoreductase (glycerone-forming) Sources: RHEA:12753 Relationships: is_a oxidoreductase activity, acting on the CH-OH group of donors, NAD or NADP as acceptor [GO:0016616]